{
  "gene_name": "Fatty acid CoA ligase Acsl3",
  "gene_symbol": "ACSL3",
  "term_label": "endoplasmic reticulum",
  "gene": "UniProtKB:O95573",
  "term_id": "GO:0005783"
}